notochord formation [GO:0014028] (biological process) Sources: GOC:dh, GOC:ef Definition: The formation of the notochord from the chordamesoderm. The notochord is composed of large cells packed within a firm connective tissue sheath and is found in all chordates at the ventral surface of the neural tube. In vertebrates, the notochord contributes to the vertebral column. Relationships: is a type of anatomical structure formation involved in morphogenesis [GO:0048646]; is part of nervous system development [GO:0007399]; is part of GO:0048570